{
  "term_label": "Unknown molecular function",
  "term_id": "UNKNOWN:0001",
  "gene_name": "Centrosomal protein of 97 kDa",
  "gene": "UniProtKB:Q8IW35",
  "gene_symbol": "CEP97"
}